energy derivation by oxidation of reduced inorganic compounds [GO:0015975] (biological process) Subtypes: methanogenesis [GO:0015948], lead sulfide oxidation [GO:0019327], GO:0019331, aerobic respiration, using nitrite as electron donor [GO:0019332], aerobic respiration, using ammonia as electron donor [GO:0019409], aerobic respiration, using carbon monoxide as electron donor [GO:0019410], aerobic respiration, using ferrous ions as electron donor [GO:0019411], aerobic respiration, using hydrogen as electron donor [GO:0019412], aerobic respiration, using sulfur or sulfate as electron donor [GO:0019414], aerobic respiration, using arsenite as electron donor [GO:0043554] Sources: GOC:mah Definition: The chemical reactions and pathways by which a cell derives energy from inorganic compounds; results in the oxidation of the compounds from which energy is released. Relationships: is a type of generation of precursor metabolites and energy [GO:0006091] Also known as: chemolithotrophie, chemolithotrophy, lithotrophy